{
  "term_label": "transcription regulator complex",
  "gene": "UniProtKB:Q2VWA4",
  "term_id": "GO:0005667",
  "gene_symbol": "SKOR2",
  "gene_name": "SKI family transcriptional corepressor 2"
}